{
  "gene_symbol": "PDCL3",
  "term_label": "protein folding chaperone",
  "gene_name": "Phosducin-like protein 3",
  "term_id": "GO:0044183",
  "gene": "UniProtKB:Q9H2J4"
}